negative regulation of steroid biosynthetic process [GO:0010894] (biological process) Relationships: is a type of negative regulation of steroid metabolic process [GO:0045939]; is a type of regulation of steroid biosynthetic process [GO:0050810]; is a type of negative regulation of lipid biosynthetic process [GO:0051055]; negatively regulates steroid biosynthetic process [GO:0006694] Sources: GOC:BHF, GOC:tb Definition: Any process that decreases the frequency, rate or extent of the chemical reactions and pathways resulting in the formation of steroids, compounds with a 1,2,cyclopentanoperhydrophenanthrene nucleus. Subtypes: negative regulation of vitamin D biosynthetic process [GO:0010957], GO:0070858, GO:0090032, GO:0106119, GO:1900841, negative regulation of androst-4-ene-3,17-dione biosynthetic process [GO:1903455], negative regulation of estrogen biosynthetic process [GO:1904077], negative regulation of androgen biosynthetic process [GO:2000180], negative regulation of progesterone biosynthetic process [GO:2000183], negative regulation of testosterone biosynthetic process [GO:2000225]